{
  "gene": "UniProtKB:Q9H0B6",
  "gene_symbol": "KLC2",
  "term_id": "GO:0007018",
  "gene_name": "Kinesin light chain 2",
  "term_label": "microtubule-based movement"
}